{
  "gene": "UniProtKB:Q9NZQ9",
  "term_label": "actin filament organization",
  "gene_symbol": "TMOD4",
  "term_id": "GO:0007015",
  "gene_name": "Tropomodulin-4"
}